{
  "term_id": "UNKNOWN:0002",
  "gene_symbol": "TEX47",
  "gene_name": "Testis-expressed protein 47",
  "term_label": "Unknown biological process",
  "gene": "UniProtKB:Q8TBZ9"
}